{
  "term_id": "UNKNOWN:0002",
  "gene": "UniProtKB:Q9HAF1",
  "gene_name": "Chromatin modification-related protein MEAF6",
  "term_label": "Unknown biological process",
  "gene_symbol": "MEAF6"
}